regulation of vegetative meristem growth [GO:0010083] (biological process) Sources: GOC:tb Definition: Any process involved in maintaining the size and shape of a vegetative meristem. Relationships: is a type of regulation of meristem growth [GO:0010075]; is a type of regulation of developmental vegetative growth [GO:1905613]; regulates GO:0010448 Also known as: regulation of vegetative meristem size